{
  "term_label": "Unknown molecular function",
  "gene_symbol": "NDUFAF5",
  "gene_name": "Arginine-hydroxylase NDUFAF5, mitochondrial",
  "gene": "UniProtKB:Q5TEU4",
  "term_id": "UNKNOWN:0001"
}